{
  "gene_name": "E3 ubiquitin-protein ligase TRIM21",
  "term_label": "regulation of gene expression",
  "term_id": "GO:0010468",
  "gene_symbol": "TRIM21",
  "gene": "UniProtKB:P19474"
}